{
  "gene_name": "Phosphatidylinositol phosphatase PTPRQ",
  "term_label": "receptor complex",
  "term_id": "GO:0043235",
  "gene": "UniProtKB:Q9UMZ3",
  "gene_symbol": "PTPRQ"
}